{
  "gene": "UniProtKB:P17019",
  "gene_symbol": "ZNF708",
  "gene_name": "Zinc finger protein 708",
  "term_label": "nucleus",
  "term_id": "GO:0005634"
}